{
  "term_label": "neurotransmitter receptor activity involved in regulation of postsynaptic cytosolic calcium ion concentration",
  "term_id": "GO:0099583",
  "gene": "UniProtKB:P41594",
  "gene_symbol": "GRM5",
  "gene_name": "Metabotropic glutamate receptor 5"
}